G protein-coupled purinergic receptor signaling pathway [GO:0035588] (biological process) Definition: A G protein-coupled receptor signaling pathway initiated by an extracellular purine or purine derivative binding to its receptor, and ending with the regulation of a downstream cellular process. Subtypes: GO:0001973 Relationships: is a type of G protein-coupled receptor signaling pathway [GO:0007186]; is a type of purinergic nucleotide receptor signaling pathway [GO:0035590] References: PMID:9755289 Sources: GOC:BHF Also known as: G-protein coupled purinergic receptor signaling pathway, G-protein coupled purinergic receptor signalling pathway